{
  "gene_name": "Putative transcription factor Ovo-like 1",
  "term_label": "RNA polymerase II cis-regulatory region sequence-specific DNA binding",
  "gene": "UniProtKB:O14753",
  "gene_symbol": "OVOL1",
  "term_id": "GO:0000978"
}